{
  "term_id": "GO:0005615",
  "gene_symbol": "OXT",
  "gene": "UniProtKB:P01178",
  "term_label": "extracellular space",
  "gene_name": "Oxytocin-neurophysin 1"
}